{
  "term_label": "mitotic spindle",
  "gene": "UniProtKB:A4D256",
  "gene_name": "Dual specificity protein phosphatase CDC14C",
  "gene_symbol": "CDC14C",
  "term_id": "GO:0072686"
}